leukocyte differentiation [GO:0002521] (biological process) Regulation: regulated by regulation of leukocyte differentiation [GO:1902105]; negatively regulated by negative regulation of leukocyte differentiation [GO:1902106]; positively regulated by positive regulation of leukocyte differentiation [GO:1902107] Also known as: immune cell differentiation, leucocyte differentiation References: PMID:16551264 Sources: CL:0000738, GOC:add Subtypes: myeloid leukocyte differentiation [GO:0002573], mononuclear cell differentiation [GO:1903131] Relationships: is a type of GO:0030154; is part of GO:0030097 Definition: The process in which a relatively unspecialized hemopoietic precursor cell acquires the specialized features of a leukocyte. A leukocyte is an achromatic cell of the myeloid or lymphoid lineages capable of ameboid movement, found in blood or other tissue.